{
  "term_label": "endosome",
  "gene_name": "Leptin receptor overlapping transcript-like 1",
  "gene_symbol": "LEPROTL1",
  "term_id": "GO:0005768",
  "gene": "UniProtKB:O95214"
}